{
  "gene_symbol": "CCL7",
  "term_id": "GO:0048020",
  "gene": "UniProtKB:P80098",
  "term_label": "CCR chemokine receptor binding",
  "gene_name": "C-C motif chemokine 7"
}